{
  "term_label": "lysosome",
  "gene_symbol": "ACP2",
  "gene_name": "Lysosomal acid phosphatase",
  "term_id": "GO:0005764",
  "gene": "UniProtKB:P11117"
}